primary plasmodesma [GO:0009550] (cellular component) Relationships: is a type of plasmodesma [GO:0009506] Definition: A plasmodesma that consists of a simple, single channel; found predominantly in young tissue and formed as a function of cell plate formation during cytokinesis. Also known as: simple plasmodesma References: PMID:15012255